establishment of protein localization to mast cell secretory granule [GO:0033369] (biological process) Definition: The directed movement of a protein to a location within a secretory granule in a mast cell. Relationships: is a type of intracellular protein transport [GO:0006886]; is part of GO:0033367 Also known as: establishment of protein localisation in mast cell secretory granule, establishment of protein localization in mast cell secretory granule Subtypes: establishment of protease localization to mast cell secretory granule [GO:0033372] Sources: GOC:mah